{
  "gene_symbol": "SHC4",
  "gene_name": "SHC-transforming protein 4",
  "term_id": "GO:0030971",
  "gene": "UniProtKB:Q6S5L8",
  "term_label": "receptor tyrosine kinase binding"
}